{
  "term_id": "GO:0005794",
  "term_label": "Golgi apparatus",
  "gene": "UniProtKB:U3KPV4",
  "gene_symbol": "A3GALT2",
  "gene_name": "Alpha-1,3-galactosyltransferase 2"
}